{
  "term_id": "GO:0035999",
  "term_label": "tetrahydrofolate interconversion",
  "gene_symbol": "MTHFD2L",
  "gene_name": "Bifunctional methylenetetrahydrofolate dehydrogenase_cyclohydrolase 2, mitochondrial",
  "gene": "UniProtKB:Q9H903"
}